{
  "gene": "UniProtKB:Q96EK5",
  "gene_symbol": "KIFBP",
  "term_label": "Unknown cellular component",
  "gene_name": "KIF-binding protein",
  "term_id": "UNKNOWN:0003"
}